{
  "gene_symbol": "HIPK2",
  "gene_name": "Homeodomain-interacting protein kinase 2",
  "term_id": "GO:0016605",
  "term_label": "PML body",
  "gene": "UniProtKB:Q9H2X6"
}